{
  "gene_symbol": "DSN1",
  "term_label": "Unknown molecular function",
  "gene": "UniProtKB:Q9H410",
  "gene_name": "Kinetochore-associated protein DSN1 homolog",
  "term_id": "UNKNOWN:0001"
}